{
  "term_label": "plasma membrane",
  "gene_symbol": "SIGLEC8",
  "gene_name": "Sialic acid-binding Ig-like lectin 8",
  "gene": "UniProtKB:Q9NYZ4",
  "term_id": "GO:0005886"
}